regulation of relaxation of muscle [GO:1901077] (biological process) Definition: Any process that modulates the frequency, rate or extent of relaxation of muscle. Sources: GOC:TermGenie Relationships: is a type of regulation of muscle system process [GO:0090257]; regulates relaxation of muscle [GO:0090075] Subtypes: negative regulation of relaxation of muscle [GO:1901078], GO:1901079, GO:1901080, regulation of relaxation of cardiac muscle [GO:1901897]